negative regulation of tumor necrosis factor-mediated signaling pathway [GO:0010804] (biological process) Relationships: is a type of negative regulation of cytokine-mediated signaling pathway [GO:0001960]; is a type of regulation of tumor necrosis factor-mediated signaling pathway [GO:0010803]; negatively regulates tumor necrosis factor-mediated signaling pathway [GO:0033209] Sources: GOC:dph, GOC:tb Also known as: negative regulation of TNF signaling, negative regulation of TNF-mediated signaling pathway, negative regulation of tumor necrosis factor-mediated signalling pathway Definition: Any process that decreases the rate or extent of the tumor necrosis factor-mediated signaling pathway. The tumor necrosis factor-mediated signaling pathway is the series of molecular signals generated as a consequence of tumor necrosis factor binding to a cell surface receptor.